regulation of protein polyglycylation [GO:1903344] (biological process) Definition: Any process that modulates the frequency, rate or extent of protein polyglycylation. Subtypes: negative regulation of protein polyglycylation [GO:1903345], positive regulation of protein polyglycylation [GO:1903346] Relationships: is a type of regulation of protein modification process [GO:0031399]; regulates GO:0018094 Sources: GOC:TermGenie, GOC:sart, GO_REF:0000058